{
  "term_label": "cell surface",
  "gene_name": "T-cell surface glycoprotein CD8 beta chain",
  "gene": "UniProtKB:P10966",
  "term_id": "GO:0009986",
  "gene_symbol": "CD8B"
}